double-stranded DNA 5'-3' DNA exonuclease activity [GO:0051908] (molecular function) Relationships: is a type of GO:0008309; is a type of 5'-3' DNA exonuclease activity [GO:0035312] Also known as: double-stranded DNA 5'-3' exodeoxyribonuclease activity, double-stranded DNA specific 5'-3' exodeoxyribonuclease activity Sources: GOC:ai Definition: Catalysis of the sequential cleavage of mononucleotides from a free 5' terminus of a double-stranded DNA molecule.